{
  "term_id": "GO:2000643",
  "gene": "UniProtKB:P15311",
  "gene_symbol": "EZR",
  "term_label": "positive regulation of early endosome to late endosome transport",
  "gene_name": "Ezrin"
}